regulation of hair cycle [GO:0042634] (biological process) Definition: Any process that modulates the frequency, rate or extent of the cyclical phases of growth (anagen), regression (catagen), quiescence (telogen), and shedding (exogen) in the life of a hair. Relationships: is a type of regulation of multicellular organismal process [GO:0051239]; regulates hair cycle [GO:0042633] Subtypes: positive regulation of hair cycle [GO:0042635], negative regulation of hair cycle [GO:0042636], regulation of hair follicle development [GO:0051797] References: PMID:12230507 Sources: GOC:go_curators